DNA N6-methyladenine demethylase activity [GO:0141131] (molecular function) Sources: RHEA:49524 Relationships: is a type of 2-oxoglutarate-dependent dioxygenase activity [GO:0016706]; is a type of DNA demethylase activity [GO:0035514] Definition: Catalysis of the reaction: 2-oxoglutarate + an N6-methyl-2'-deoxyadenosine in DNA + O2 = a 2'-deoxyadenosine in DNA + CO2 + formaldehyde + succinate. Also known as: DNA N(6)-methyladenine demethylase activity